{
  "term_id": "UNKNOWN:0002",
  "term_label": "Unknown biological process",
  "gene": "UniProtKB:Q99437",
  "gene_symbol": "ATP6V0B",
  "gene_name": "V-type proton ATPase 21 kDa proteolipid subunit c''"
}